{
  "gene_name": "Golgin subfamily A member 2",
  "gene_symbol": "GOLGA2",
  "term_id": "GO:0005801",
  "term_label": "cis-Golgi network",
  "gene": "UniProtKB:Q08379"
}